negative regulation of hepatocyte growth factor production [GO:0032686] (biological process) Also known as: down regulation of hepatocyte growth factor production, down-regulation of hepatocyte growth factor production, downregulation of hepatocyte growth factor production, negative regulation of HGF production, negative regulation of scatter factor production, inhibition of hepatocyte growth factor production, negative regulation of hepatocyte growth factor biosynthetic process References: PMID:1838014 Sources: GOC:mah Definition: Any process that stops, prevents, or reduces the frequency, rate, or extent of hepatocyte growth factor production. Relationships: is a type of negative regulation of cytokine production [GO:0001818]; is a type of GO:0032646; is a type of GO:0051248; negatively regulates GO:0032605